{
  "term_id": "GO:0000049",
  "term_label": "tRNA binding",
  "gene_name": "Eukaryotic translation initiation factor 2 subunit 3B",
  "gene_symbol": "EIF2S3B",
  "gene": "UniProtKB:Q2VIR3"
}